cellular response to lipoic acid [GO:1903443] (biological process) Relationships: is_a cellular response to fatty acid [GO:0071398]; is a type of response to lipoic acid [GO:1903442] References: PMID:23232760 Sources: GOC:TermGenie, GOC:sl, GO_REF:0000071 Definition: Any process that results in a change in state or activity of a cell (in terms of movement, secretion, enzyme production, gene expression, etc.) as a result of a lipoic acid stimulus.